{
  "gene_symbol": "FHIT",
  "gene_name": "Bis(5'-adenosyl)-triphosphatase",
  "gene": "UniProtKB:P49789",
  "term_label": "intrinsic apoptotic signaling pathway by p53 class mediator",
  "term_id": "GO:0072332"
}